{
  "term_label": "RNA polymerase II cis-regulatory region sequence-specific DNA binding",
  "gene_name": "Transcription factor p65",
  "gene": "UniProtKB:Q04206",
  "term_id": "GO:0000978",
  "gene_symbol": "RELA"
}